{
  "term_label": "late endosome to vacuole transport via multivesicular body sorting pathway",
  "term_id": "GO:0032511",
  "gene": "UniProtKB:O95214",
  "gene_name": "Leptin receptor overlapping transcript-like 1",
  "gene_symbol": "LEPROTL1"
}